{
  "term_label": "mitochondrial outer membrane",
  "gene": "UniProtKB:Q16611",
  "gene_symbol": "BAK1",
  "term_id": "GO:0005741",
  "gene_name": "Bcl-2 homologous antagonist_killer"
}